interleukin-13 receptor binding [GO:0005144] (MF) Also known as: IL-13, interleukin-13 receptor ligand Definition: Binding to an interleukin-13 receptor. Sources: GOC:ai Relationships: is a type of cytokine receptor binding [GO:0005126]